{
  "term_label": "morphogenesis of an epithelium",
  "gene": "UniProtKB:P35527",
  "gene_symbol": "KRT9",
  "gene_name": "Keratin, type I cytoskeletal 9",
  "term_id": "GO:0002009"
}